ribosomal small subunit assembly [GO:0000028] (biological process) References: PMID:30467428 Sources: GOC:jl Also known as: 30S ribosomal subunit assembly, 40S ribosomal subunit assembly Definition: The aggregation, arrangement and bonding together of constituent RNAs and proteins to form the small ribosomal subunit. Subtypes: cytosolic small ribosomal subunit assembly [GO:0180025], mitochondrial small ribosomal subunit assembly [GO:0180026] Relationships: is a type of GO:0022618; is part of GO:0042255; is part of ribosomal small subunit biogenesis [GO:0042274]